{
  "gene": "UniProtKB:Q9BS16",
  "gene_name": "Centromere protein K",
  "gene_symbol": "CENPK",
  "term_id": "UNKNOWN:0001",
  "term_label": "Unknown molecular function"
}